{
  "gene_name": "Krueppel-like factor 13",
  "gene_symbol": "KLF13",
  "term_label": "nucleus",
  "gene": "UniProtKB:Q9Y2Y9",
  "term_id": "GO:0005634"
}